calcium-dependent protein kinase inhibitor activity [GO:0008427] (molecular function) Definition: Binds to and stops, prevents or reduces the activity of a calcium-dependent protein kinase. Sources: GOC:mah Relationships: is a type of GO:0010858; is a type of protein serine/threonine kinase inhibitor activity [GO:0030291]; negatively regulates calcium-dependent protein serine/threonine kinase activity [GO:0009931]